{
  "gene_name": "TOM1-like protein 1",
  "gene_symbol": "TOM1L1",
  "gene": "UniProtKB:O75674",
  "term_id": "GO:0030276",
  "term_label": "clathrin binding"
}